spermathecum morphogenesis [GO:0035211] (biological process) Definition: The process in which the anatomical structures of a spermathecum, a sperm storage organ, are generated and organized. Paired spermathecae lie at the anterior end of the insect uterus on the dorsal side. Each spermatheca consists of an oval shaped capsule, connected to the uterus by a spermathecal stalk. Relationships: is a type of animal organ morphogenesis [GO:0009887] References: PMID:12679097 Note: See also the fly_anatomy.ontology term 'spermathecum ; FBbt:00004921'.